{
  "term_label": "endomembrane system",
  "gene": "UniProtKB:O94876",
  "gene_symbol": "TMCC1",
  "gene_name": "Transmembrane and coiled-coil domains protein 1",
  "term_id": "GO:0012505"
}